{
  "term_id": "GO:0098554",
  "gene_name": "Signal peptide peptidase-like 2A",
  "gene": "UniProtKB:Q8TCT8",
  "term_label": "cytoplasmic side of endoplasmic reticulum membrane",
  "gene_symbol": "SPPL2A"
}